{
  "term_id": "GO:0005886",
  "gene_name": "Syntaxin-1B",
  "gene": "UniProtKB:P61266",
  "gene_symbol": "STX1B",
  "term_label": "plasma membrane"
}